{
  "gene_name": "Acyl-coenzyme A thioesterase 9, mitochondrial",
  "term_label": "fatty acyl-CoA hydrolase activity",
  "gene": "UniProtKB:Q9Y305",
  "term_id": "GO:0047617",
  "gene_symbol": "ACOT9"
}